cell communication by electrical coupling [GO:0010644] (biological process) Subtypes: cell communication by electrical coupling involved in cardiac conduction [GO:0086064] Sources: GOC:dph, GOC:kmv, GOC:tb Regulation: regulated by GO:0010649; positively regulated by positive regulation of cell communication by electrical coupling [GO:0010650]; negatively regulated by GO:0010651 Relationships: is a type of cell communication [GO:0007154] Definition: The process that mediates signaling interactions between one cell and another cell by transfer of current between their adjacent cytoplasms via intercellular protein channels.